negative regulation of protein neddylation [GO:2000435] (biological process) Also known as: negative regulation of RUB1-protein conjugation Sources: GOC:obol Relationships: is a type of GO:1903321; is a type of regulation of protein neddylation [GO:2000434]; negatively regulates protein neddylation [GO:0045116] Definition: Any process that stops, prevents or reduces the frequency, rate or extent of protein neddylation.